{
  "gene_symbol": "ZDHHC4",
  "gene": "UniProtKB:Q9NPG8",
  "gene_name": "Palmitoyltransferase ZDHHC4",
  "term_id": "GO:0006612",
  "term_label": "protein targeting to membrane"
}